{
  "gene_symbol": "RPA4",
  "term_label": "telomeric DNA binding",
  "gene_name": "Replication protein A 30 kDa subunit",
  "term_id": "GO:0042162",
  "gene": "UniProtKB:Q13156"
}